{
  "gene_symbol": "HLA-DQB1",
  "term_label": "positive regulation of T cell activation",
  "term_id": "GO:0050870",
  "gene_name": "HLA class II histocompatibility antigen, DQ beta 1 chain",
  "gene": "UniProtKB:P01920"
}